{
  "gene_symbol": "DOCK9",
  "gene_name": "Dedicator of cytokinesis protein 9",
  "term_id": "GO:0035023",
  "gene": "UniProtKB:Q9BZ29",
  "term_label": "regulation of Rho protein signal transduction"
}